{
  "gene_name": "LIM and senescent cell antigen-like-containing domain protein 4",
  "gene": "UniProtKB:P0CW20",
  "gene_symbol": "LIMS4",
  "term_id": "UNKNOWN:0003",
  "term_label": "Unknown cellular component"
}